{
  "gene_symbol": "HCCS",
  "term_id": "GO:0004408",
  "term_label": "holocytochrome-c synthase activity",
  "gene": "UniProtKB:P53701",
  "gene_name": "Holocytochrome c-type synthase"
}